{
  "term_label": "RNA polymerase II cis-regulatory region sequence-specific DNA binding",
  "term_id": "GO:0000978",
  "gene_symbol": "NKX6-3",
  "gene_name": "Homeobox protein Nkx-6.3",
  "gene": "UniProtKB:A6NJ46"
}